{
  "term_id": "UNKNOWN:0002",
  "term_label": "Unknown biological process",
  "gene_symbol": "C3orf20",
  "gene": "UniProtKB:Q8ND61",
  "gene_name": "Uncharacterized protein C3orf20"
}